{
  "gene_name": "Collagen alpha-1(I) chain",
  "gene_symbol": "COL1A1",
  "term_id": "UNKNOWN:0003",
  "term_label": "Unknown cellular component",
  "gene": "UniProtKB:P02452"
}